{
  "gene": "UniProtKB:Q53FT3",
  "gene_name": "Protein Hikeshi",
  "term_label": "protein import into nucleus",
  "gene_symbol": "HIKESHI",
  "term_id": "GO:0006606"
}